{
  "term_label": "galactokinase activity",
  "gene": "UniProtKB:P51570",
  "gene_symbol": "GALK1",
  "term_id": "GO:0004335",
  "gene_name": "Galactokinase"
}